{
  "gene_symbol": "PORCN",
  "gene_name": "Protein-serine O-palmitoleoyltransferase porcupine",
  "gene": "UniProtKB:Q9H237",
  "term_id": "GO:1990698",
  "term_label": "palmitoleoyltransferase activity"
}